{
  "gene_symbol": "NAPG",
  "term_id": "GO:0019905",
  "gene_name": "Gamma-soluble NSF attachment protein",
  "term_label": "syntaxin binding",
  "gene": "UniProtKB:Q99747"
}